{
  "term_id": "GO:0007186",
  "gene_symbol": "RGS9BP",
  "gene": "UniProtKB:Q6ZS82",
  "term_label": "G protein-coupled receptor signaling pathway",
  "gene_name": "Regulator of G-protein signaling 9-binding protein"
}